{
  "gene_name": "Fer3-like protein",
  "gene": "UniProtKB:Q96RJ6",
  "term_id": "GO:0006357",
  "gene_symbol": "FERD3L",
  "term_label": "regulation of transcription by RNA polymerase II"
}